{
  "gene_name": "TLR4 interactor with leucine rich repeats",
  "term_label": "lipopolysaccharide receptor complex",
  "term_id": "GO:0046696",
  "gene_symbol": "TRIL",
  "gene": "UniProtKB:Q7L0X0"
}